{
  "gene": "UniProtKB:Q5QJ74",
  "gene_name": "Tubulin-specific chaperone cofactor E-like protein",
  "term_id": "GO:0007023",
  "gene_symbol": "TBCEL",
  "term_label": "post-chaperonin tubulin folding pathway"
}